{
  "gene_symbol": "CHSY1",
  "term_label": "Unknown cellular component",
  "term_id": "UNKNOWN:0003",
  "gene": "UniProtKB:Q86X52",
  "gene_name": "Chondroitin sulfate synthase 1"
}